ecdysteroid metabolic process [GO:0045455] (biological process) Definition: The chemical reactions and pathways involving ecdysteroids, a group of polyhydroxylated ketosteroids ubiquitous in insects and other arthropods, in which they initiate post-embryonic development, including the metamorphosis of immature forms and the development of the reproductive system and the maturation of oocytes in adult females. Sources: ISBN:0198506732 Also known as: ecdysteroid metabolism Relationships: is a type of GO:0008202; is a type of ketone metabolic process [GO:0042180]; is a type of hormone metabolic process [GO:0042445]; is part of GO:0002165 Subtypes: ecdysone metabolic process [GO:0008205], ecdysteroid biosynthetic process [GO:0045456], ecdysteroid catabolic process [GO:0046344] Regulation: regulated by regulation of ecdysteroid metabolic process [GO:0007553]